N-terminal peptidyl-alanine methylation [GO:0018011] (biological process) Definition: The methylation of the N-terminal alanine of proteins. Subtypes: GO:0018012 Relationships: is a type of N-terminal protein amino acid methylation [GO:0006480]; is a type of GO:0018194 Sources: RESID:AA0061, RESID:AA0062